{
  "gene_name": "Putative BPES syndrome breakpoint region protein",
  "term_id": "UNKNOWN:0003",
  "gene_symbol": "BPESC1",
  "gene": "UniProtKB:Q9GZL8",
  "term_label": "Unknown cellular component"
}